{
  "gene": "UniProtKB:P43088",
  "gene_symbol": "PTGFR",
  "term_label": "prostaglandin F receptor activity",
  "term_id": "GO:0004958",
  "gene_name": "Prostaglandin F2-alpha receptor"
}